{
  "gene_name": "Putative dispanin subfamily A member 2d",
  "gene": "UniProtKB:C9JQL5",
  "term_id": "GO:0045071",
  "gene_symbol": "C9JQL5",
  "term_label": "negative regulation of viral genome replication"
}